negative regulation of acetylcholine uptake [GO:0051632] (biological process) Also known as: down regulation of acetylcholine uptake, down-regulation of acetylcholine uptake, downregulation of acetylcholine uptake, negative regulation of acetylcholine import Sources: GOC:ai Definition: Any process that stops, prevents, or reduces the frequency, rate or extent of the directed movement of acetylcholine into a cell. Relationships: is a type of regulation of acetylcholine uptake [GO:0051631]; is a type of negative regulation of amine transport [GO:0051953]; negatively regulates acetylcholine uptake [GO:0051630] Subtypes: inhibition of acetylcholine uptake [GO:0051634]